pre-miRNA 3'-end processing [GO:0044747] (biological process) Definition: Any process involved in forming distinct miRNA isoforms from a mature miRNA that differ at their 3'-ends. Relationships: is a type of GO:0031054; is a type of regulatory ncRNA 3'-end processing [GO:0043628]; is part of miRNA processing [GO:0035196] Also known as: miRNA 3' end terminal trimming, miRNA 3'-end processing, miRNA trimming, mature miRNA 3'-end processing References: PMID:22055292, PMID:22055293